{
  "gene_symbol": "DCT",
  "gene_name": "L-dopachrome tautomerase",
  "term_label": "ventricular zone neuroblast division",
  "gene": "UniProtKB:P40126",
  "term_id": "GO:0021847"
}